{
  "gene_symbol": "TAF9",
  "gene": "UniProtKB:Q16594",
  "term_label": "RNA polymerase II general transcription initiation factor activity",
  "gene_name": "Transcription initiation factor TFIID subunit 9",
  "term_id": "GO:0016251"
}